IgA receptor activity [GO:0019766] (MF) Subtypes: high-affinity IgA receptor activity [GO:0002170], low-affinity IgA receptor activity [GO:0002171] Definition: Combining with an immunoglobulin of an IgA isotype via the Fc region, and transmitting the signal from one side of the membrane to the other to initiate a change in cell activity. Sources: GOC:add, GOC:signaling, ISBN:0781735149 Relationships: is a type of immunoglobulin receptor activity [GO:0019763]; has part IgA binding [GO:0019862]